L-isoleucine catabolic process [GO:0006550] (biological process) Definition: The chemical reactions and pathways resulting in the breakdown of L-isoleucine, (2R*,3R*)-2-amino-3-methylpentanoic acid. Sources: GOC:ai Also known as: isoleucine breakdown, isoleucine catabolism, isoleucine degradation Relationships: is a type of isoleucine metabolic process [GO:0006549]; is a type of branched-chain amino acid catabolic process [GO:0009083]; is a type of L-amino acid catabolic process [GO:0170035]; is_a proteinogenic amino acid catabolic process [GO:0170040]